{
  "gene": "UniProtKB:Q9BUL8",
  "term_id": "GO:0090168",
  "gene_name": "Programmed cell death protein 10",
  "gene_symbol": "PDCD10",
  "term_label": "Golgi reassembly"
}